{
  "gene": "UniProtKB:Q92820",
  "term_id": "GO:0046900",
  "gene_name": "Gamma-glutamyl hydrolase",
  "term_label": "tetrahydrofolylpolyglutamate metabolic process",
  "gene_symbol": "GGH"
}